{
  "gene": "UniProtKB:P07306",
  "gene_symbol": "ASGR1",
  "gene_name": "Asialoglycoprotein receptor 1",
  "term_id": "GO:0042806",
  "term_label": "fucose binding"
}